{
  "gene_name": "Mothers against decapentaplegic homolog 1",
  "term_label": "SMAD protein signal transduction",
  "gene_symbol": "SMAD1",
  "term_id": "GO:0060395",
  "gene": "UniProtKB:Q15797"
}